{
  "term_id": "GO:0003730",
  "gene_symbol": "IGF2BP1",
  "gene": "UniProtKB:Q9NZI8",
  "term_label": "mRNA 3'-UTR binding",
  "gene_name": "Insulin-like growth factor 2 mRNA-binding protein 1"
}